{
  "gene_symbol": "SCML1",
  "term_label": "histone binding",
  "gene": "UniProtKB:Q9UN30",
  "gene_name": "Sex comb on midleg-like protein 1",
  "term_id": "GO:0042393"
}